negative regulation of glucokinase activity [GO:0033132] (biological process) Sources: GOC:mah Relationships: is_a GO:0033673; negatively regulates GO:0004340 Definition: Any process that stops, prevents, or reduces the frequency, rate or extent of glucokinase activity, the catalysis of the transfer of a phosphate group, usually from ATP, to a glucose molecule. Also known as: down regulation of glucokinase activity, down-regulation of glucokinase activity, downregulation of glucokinase activity, glucokinase inhibitor, inhibition of glucokinase activity